dichloromethane metabolic process [GO:0018900] (biological process) Definition: The chemical reactions and pathways involving dichloromethane, a dichlorinated derivative of methane. It is a colorless organic liquid with a sweet, chloroform-like odor, often used as a paint remover. Sources: UM-BBD_pathwayID:dcm Also known as: dichloromethane metabolism Relationships: is a type of halogenated hydrocarbon metabolic process [GO:0042197]